positive regulation of antibody-dependent cellular cytotoxicity [GO:0001815] (biological process) Also known as: positive regulation of antibody dependent cell death, positive regulation of antibody dependent cell killing, positive regulation of antibody-dependent cell death, positive regulation of antibody-dependent cell killing, up regulation of antibody-dependent cellular cytotoxicity, up-regulation of antibody-dependent cellular cytotoxicity, upregulation of antibody-dependent cellular cytotoxicity, activation of antibody-dependent cellular cytotoxicity, stimulation of antibody-dependent cellular cytotoxicity Sources: GOC:add, ISBN:0781735149 Definition: Any process that activates or increases the frequency, rate or extent of antibody-dependent cellular cytotoxicity. Relationships: is a type of positive regulation of type IIa hypersensitivity [GO:0001798]; is a type of regulation of antibody-dependent cellular cytotoxicity [GO:0001813]; is a type of positive regulation of leukocyte mediated cytotoxicity [GO:0001912]; positively regulates antibody-dependent cellular cytotoxicity [GO:0001788]